{
  "gene_name": "Disintegrin and metalloproteinase domain-containing protein 2",
  "term_label": "plasma membrane",
  "gene_symbol": "ADAM2",
  "term_id": "GO:0005886",
  "gene": "UniProtKB:Q99965"
}